{
  "term_id": "GO:0061630",
  "gene_symbol": "UBR3",
  "gene": "UniProtKB:Q6ZT12",
  "term_label": "ubiquitin protein ligase activity",
  "gene_name": "E3 ubiquitin-protein ligase UBR3"
}